{
  "term_label": "Unknown biological process",
  "gene": "UniProtKB:P0CF75",
  "gene_name": "Endogenous Bornavirus-like nucleoprotein 1",
  "gene_symbol": "EBLN1",
  "term_id": "UNKNOWN:0002"
}